{
  "gene": "UniProtKB:P54727",
  "gene_name": "UV excision repair protein RAD23 homolog B",
  "term_id": "GO:0070628",
  "gene_symbol": "RAD23B",
  "term_label": "proteasome binding"
}